{
  "gene_name": "Methyltransferase-like 26",
  "term_label": "Unknown biological process",
  "gene": "UniProtKB:Q96S19",
  "gene_symbol": "METTL26",
  "term_id": "UNKNOWN:0002"
}